{
  "term_label": "cytosol",
  "gene_name": "Segment polarity protein dishevelled homolog DVL-3",
  "gene": "UniProtKB:Q92997",
  "gene_symbol": "DVL3",
  "term_id": "GO:0005829"
}